regulation of vesicle fusion [GO:0031338] (biological process) Relationships: is a type of regulation of organelle organization [GO:0033043]; is a type of regulation of vesicle-mediated transport [GO:0060627]; regulates GO:0006906 Definition: Any process that modulates the frequency, rate or extent of vesicle fusion. Sources: GOC:mah Subtypes: negative regulation of vesicle fusion [GO:0031339], positive regulation of vesicle fusion [GO:0031340], regulation of synaptic vesicle fusion to presynaptic active zone membrane [GO:0031630], regulation of Golgi vesicle fusion to target membrane [GO:0048214], regulation of vesicle fusion with Golgi apparatus [GO:0106214], regulation of endosomal vesicle fusion [GO:1905364]